inductive cell migration [GO:0040039] (BP) Relationships: is a type of cell migration [GO:0016477] Sources: ISBN:087969307X, ISBN:0879694882 Definition: Migration of a cell in a multicellular organism that, having changed its location, is required to induce normal properties in one or more cells at its new location. An example of this would be the distal tip cells of Caenorhabditis elegans.